{
  "term_label": "signal transduction",
  "gene": "UniProtKB:Q86Y07",
  "gene_symbol": "VRK2",
  "term_id": "GO:0007165",
  "gene_name": "Serine_threonine-protein kinase VRK2"
}